snRNA pseudouridine synthesis [GO:0031120] (biological process) Definition: The intramolecular conversion of uridine to pseudouridine in an snRNA molecule. Sources: GOC:mah Regulation: regulated by regulation of snRNA pseudouridine synthesis [GO:1905356]; negatively regulated by negative regulation of snRNA pseudouridine synthesis [GO:1905357]; positively regulated by positive regulation of snRNA pseudouridine synthesis [GO:1905358] Relationships: is a type of GO:0001522; is a type of snRNA modification [GO:0040031]